{
  "term_label": "adherens junction",
  "term_id": "GO:0005912",
  "gene_symbol": "NECTIN1",
  "gene": "UniProtKB:Q15223",
  "gene_name": "Nectin-1"
}